{
  "gene_name": "Cerebellin-2",
  "gene": "UniProtKB:Q8IUK8",
  "gene_symbol": "CBLN2",
  "term_label": "trans-synaptic signaling, modulating synaptic transmission",
  "term_id": "GO:0099550"
}